{
  "term_label": "Unknown biological process",
  "gene": "UniProtKB:Q6ZRX8",
  "term_id": "UNKNOWN:0002",
  "gene_symbol": "Q6ZRX8",
  "gene_name": "Putative uncharacterized protein FLJ45999"
}